{
  "gene_symbol": "CGB3",
  "term_label": "hormone activity",
  "term_id": "GO:0005179",
  "gene_name": "Choriogonadotropin subunit beta 3",
  "gene": "UniProtKB:P0DN86"
}